{
  "term_id": "UNKNOWN:0001",
  "gene_name": "Solute carrier family 22 member 11",
  "term_label": "Unknown molecular function",
  "gene_symbol": "SLC22A11",
  "gene": "UniProtKB:Q9NSA0"
}